pollen wall [GO:0043667] (cellular component) References: PMID:15131249 Sources: GOC:fz Definition: The wall surrounding a mature pollen grain; a multilayered structure consisting of a pectocellulosic intine surrounded by a sporopollenin-based exine, which itself contains two layers, the inner nexine and the outer sexine. Also known as: microspore wall Relationships: is a type of external encapsulating structure [GO:0030312]